2-keto-3-deoxygluconate transmembrane transport [GO:0046411] (biological process) Relationships: is a type of GO:0015718; is a type of monosaccharide transmembrane transport [GO:0015749]; is a type of carboxylic acid transmembrane transport [GO:1905039] Also known as: 2-keto-3-deoxygluconate transport Sources: GOC:go_curators Definition: The process in which 2-keto-3-deoxygluconate is transported across a lipid bilayer, from one side of a membrane to the other.